{
  "gene_symbol": "BTNL9",
  "gene": "UniProtKB:Q6UXG8",
  "gene_name": "Butyrophilin-like protein 9",
  "term_label": "T cell receptor signaling pathway",
  "term_id": "GO:0050852"
}